cellular response to leucine starvation [GO:1990253] (biological process) Definition: Any process that results in a change in state or activity of a cell (in terms of movement, secretion, enzyme production, gene expression, etc.) as a result of deprivation of leucine. References: PMID:19033384 Relationships: is a type of GO:0034198